{
  "gene": "UniProtKB:P32418",
  "gene_symbol": "SLC8A1",
  "gene_name": "Sodium_calcium exchanger 1",
  "term_id": "GO:0098794",
  "term_label": "postsynapse"
}